maintenance of transcriptional fidelity during transcription elongation [GO:0001192] (biological process) Subtypes: maintenance of transcriptional fidelity during transcription elongation by RNA polymerase II [GO:0001193], GO:0001195 Relationships: is a type of GO:0032774; is part of DNA-templated transcription elongation [GO:0006354] Definition: Suppression of the occurrence of transcriptional errors, such as substitutions and/or insertions of nucleotides that do not correctly match the template base, during the process of transcription elongation on a DNA template. Sources: GOC:txnOH Also known as: maintenance of transcriptional fidelity during DNA-dependent transcription elongation, maintenance of transcriptional fidelity during DNA-dependent transcription elongation from bacterial-type RNA polymerase promoter, maintenance of transcriptional fidelity during DNA-templated transcription elongation, maintenance of transcriptional fidelity during DNA-templated transcription elongation from bacterial-type RNA polymerase promoter